Fas signaling pathway [GO:0036337] (biological process) References: PMID:12040174 Sources: GOC:nhn, Wikipedia:Fas_receptor Relationships: is a type of cell surface receptor signaling pathway [GO:0007166] Regulation: regulated by GO:1902044; negatively regulated by GO:1902045; RO_0002213 by positive regulation of Fas signaling pathway [GO:1902046] Definition: The series of molecular signals initiated by the binding of a ligand to a Fas receptor on the surface of the cell, and ending with the regulation of a downstream cellular process, e.g. transcription. Fas is a death domain-containing member of the tumor necrosis factor receptor (TNFR) superfamily. Also known as: Apo-1 signaling pathway, CD95 signaling pathway, Fas receptor signaling pathway, FasR signaling pathway, FAS ligand-Fas signaling pathway, Fas-FasL signaling pathway, FasL signaling pathway